cell volume homeostasis [GO:0006884] (biological process) Subtypes: GO:0009992, negative regulation of cell volume [GO:0045794], positive regulation of cell volume [GO:0045795] Relationships: is a type of regulation of cell size [GO:0008361]; is a type of cellular homeostasis [GO:0019725] Definition: Any process involved in maintaining the steady state of a cell's volume. The cell's volume refers to the three-dimensional space occupied by a cell. Sources: GOC:dph, GOC:go_curators, GOC:tb Also known as: regulation of cell volume